{
  "term_id": "GO:0005737",
  "gene_name": "Serine_threonine-protein kinase H2",
  "gene": "UniProtKB:Q96QS6",
  "term_label": "cytoplasm",
  "gene_symbol": "PSKH2"
}